indole-3-acetyl-methionine synthetase activity [GO:0102049] (molecular function) Relationships: is a type of ligase activity, forming carbon-nitrogen bonds [GO:0016879] Definition: Catalysis of the reaction: indole-3-acetate + L-methionine + ATP(4-) = H+ + indole-3-acetyl-methionine + AMP(2-) + diphosphoric acid. References: PMID:15659623 Sources: GOC:pz